{
  "gene_name": "Peroxisomal sarcosine oxidase",
  "term_label": "peroxisome",
  "gene_symbol": "PIPOX",
  "gene": "UniProtKB:Q9P0Z9",
  "term_id": "GO:0005777"
}